{
  "term_label": "box C/D methylation guide snoRNP complex",
  "gene": "UniProtKB:P22087",
  "term_id": "GO:0031428",
  "gene_symbol": "FBL",
  "gene_name": "rRNA 2'-O-methyltransferase fibrillarin"
}